{
  "gene_symbol": "RAC1",
  "gene_name": "Ras-related C3 botulinum toxin substrate 1",
  "gene": "UniProtKB:P63000",
  "term_label": "Rac protein signal transduction",
  "term_id": "GO:0016601"
}